negative regulation of sodium ion export across plasma membrane [GO:1903277] (biological process) References: PMID:17095720 Sources: GOC:BHF, GOC:TermGenie, GOC:rl, GO_REF:0000058 Relationships: is a type of GO:1902306; is a type of regulation of sodium ion export across plasma membrane [GO:1903276]; negatively regulates sodium ion export across plasma membrane [GO:0036376] Also known as: down regulation of sodium ion export from cell, down-regulation of sodium ion export from cell, downregulation of sodium ion export from cell, negative regulation of sodium ion export from cell, inhibition of sodium export, inhibition of sodium ion export, inhibition of sodium ion export from cell, down regulation of sodium export, down regulation of sodium ion export, down-regulation of sodium export, down-regulation of sodium ion export, downregulation of sodium export, downregulation of sodium ion export, negative regulation of sodium export, negative regulation of sodium ion export Definition: Any process that stops, prevents or reduces the frequency, rate or extent of sodium ion export across the plasma membrane.